{
  "gene_name": "ATPase family AAA domain-containing protein 3C",
  "gene_symbol": "ATAD3C",
  "term_id": "GO:0007005",
  "term_label": "mitochondrion organization",
  "gene": "UniProtKB:Q5T2N8"
}